{
  "gene_name": "Pro-opiomelanocortin",
  "gene_symbol": "POMC",
  "term_id": "GO:2000852",
  "gene": "UniProtKB:P01189",
  "term_label": "regulation of corticosterone secretion"
}